{
  "gene_symbol": "ZPLD1",
  "gene": "UniProtKB:Q8TCW7",
  "gene_name": "Zona pellucida-like domain-containing protein 1",
  "term_label": "Unknown molecular function",
  "term_id": "UNKNOWN:0001"
}